{
  "term_id": "UNKNOWN:0001",
  "gene_name": "Secretoglobin family 3A member 1",
  "gene_symbol": "SCGB3A1",
  "term_label": "Unknown molecular function",
  "gene": "UniProtKB:Q96QR1"
}